cyclopentanone monooxygenase activity [GO:0047799] (molecular function) Sources: EC:1.14.13.16, RHEA:15737 Relationships: is_a oxidoreductase activity, acting on paired donors, with incorporation or reduction of molecular oxygen, NAD(P)H as one donor, and incorporation of one atom of oxygen [GO:0016709] Also known as: cyclopentanone 1,2-monooxygenase activity, cyclopentanone oxygenase activity, cyclopentanone,NADPH:oxygen oxidoreductase (5-hydroxylating, lactonizing) Definition: Catalysis of the reaction: cyclopentanone + H+ + NADPH + O2 = 5-valerolactone + H2O + NADP+.